{
  "gene_symbol": "THUMPD1",
  "gene_name": "THUMP domain-containing protein 1",
  "gene": "UniProtKB:Q9NXG2",
  "term_id": "UNKNOWN:0003",
  "term_label": "Unknown cellular component"
}